{
  "gene": "UniProtKB:P18509",
  "gene_symbol": "ADCYAP1",
  "gene_name": "Pituitary adenylate cyclase-activating polypeptide",
  "term_id": "GO:0007218",
  "term_label": "neuropeptide signaling pathway"
}